{
  "term_id": "GO:0001819",
  "gene_symbol": "CD14",
  "term_label": "positive regulation of cytokine production",
  "gene": "UniProtKB:P08571",
  "gene_name": "Monocyte differentiation antigen CD14"
}